{
  "term_id": "GO:0032785",
  "gene_name": "Zinc finger CCCH domain-containing protein 8",
  "gene": "UniProtKB:Q8N5P1",
  "term_label": "negative regulation of DNA-templated transcription, elongation",
  "gene_symbol": "ZC3H8"
}